{
  "gene_name": "Helicase-like transcription factor",
  "gene_symbol": "HLTF",
  "term_label": "DNA repair",
  "gene": "UniProtKB:Q14527",
  "term_id": "GO:0006281"
}